{
  "gene": "UniProtKB:Q9UKX3",
  "gene_symbol": "MYH13",
  "term_id": "GO:0006936",
  "term_label": "muscle contraction",
  "gene_name": "Myosin-13"
}